{
  "term_id": "GO:0043161",
  "gene_name": "Seven in absentia homolog 3",
  "term_label": "proteasome-mediated ubiquitin-dependent protein catabolic process",
  "gene": "UniProtKB:Q8IW03",
  "gene_symbol": "SIAH3"
}